{
  "gene_name": "C-X-C motif chemokine 6",
  "term_id": "GO:0008009",
  "term_label": "chemokine activity",
  "gene_symbol": "CXCL6",
  "gene": "UniProtKB:P80162"
}